{
  "term_id": "UNKNOWN:0003",
  "term_label": "Unknown cellular component",
  "gene_symbol": "IQANK1",
  "gene_name": "IQ motif and ankyrin repeat domain-containing protein 1",
  "gene": "UniProtKB:A8MXQ7"
}